{
  "term_id": "GO:0048019",
  "gene_symbol": "DKK2",
  "gene": "UniProtKB:Q9UBU2",
  "term_label": "receptor antagonist activity",
  "gene_name": "Dickkopf-related protein 2"
}